{
  "gene_symbol": "BMAL1",
  "gene": "UniProtKB:O00327",
  "gene_name": "Basic helix-loop-helix ARNT-like protein 1",
  "term_label": "DNA-binding transcription factor activity, RNA polymerase II-specific",
  "term_id": "GO:0000981"
}